accessory nerve morphogenesis [GO:0021607] (biological process) Relationships: is a type of cranial nerve morphogenesis [GO:0021602]; is part of accessory nerve development [GO:0021565] Sources: GOC:cls, GOC:dgh, GOC:dph, GOC:jid, GO_REF:0000021 Definition: The process in which the anatomical structure of the accessory nerve is generated and organized. The spinal branch of this motor nerve innervates the trapezius and the sternocleidomastoid muscles. The cranial branch joins the vagus nerve and innervates the same targets as the vagus nerve. Also known as: CN XI morphogenesis